regulation of motor neuron apoptotic process [GO:2000671] (biological process) Also known as: regulation of motoneuron apoptosis, regulation of motor neuron apoptosis Definition: Any process that modulates the frequency, rate or extent of motor neuron apoptotic process. Sources: GOC:mtg_apoptosis, GOC:obol Relationships: is_a regulation of neuron apoptotic process [GO:0043523]; regulates motor neuron apoptotic process [GO:0097049] Subtypes: GO:2000672, positive regulation of motor neuron apoptotic process [GO:2000673]